{
  "term_label": "DNA-binding transcription factor activity, RNA polymerase II-specific",
  "term_id": "GO:0000981",
  "gene": "UniProtKB:Q15672",
  "gene_name": "Twist-related protein 1",
  "gene_symbol": "TWIST1"
}